{
  "gene": "UniProtKB:Q99496",
  "gene_name": "E3 ubiquitin-protein ligase RING2",
  "term_label": "ubiquitin ligase complex",
  "term_id": "GO:0000151",
  "gene_symbol": "RNF2"
}